{
  "term_label": "centriole",
  "term_id": "GO:0005814",
  "gene": "UniProtKB:Q12798",
  "gene_name": "Centrin-1",
  "gene_symbol": "CETN1"
}